{
  "term_id": "GO:0005615",
  "gene": "UniProtKB:Q9BY76",
  "gene_name": "Angiopoietin-related protein 4",
  "term_label": "extracellular space",
  "gene_symbol": "ANGPTL4"
}